{
  "gene": "UniProtKB:Q9UHP9",
  "gene_symbol": "SMPX",
  "gene_name": "Small muscular protein",
  "term_id": "GO:0005927",
  "term_label": "muscle tendon junction"
}